D-lysine 5,6-aminomutase activity [GO:0047826] (molecular function) Sources: EC:5.4.3.3 Relationships: is_a intramolecular aminotransferase activity [GO:0016869] Definition: Catalysis of the reaction: D-lysine = (2R,5S)-2,5-diaminohexanoate and (3S)-3,6-diaminohexanoate = (3S,5S)-3,5-diaminohexanoate. Also known as: adenosylcobalamin-dependent D-lysine 5,6-aminomutase activity, lysine 5,6-aminomutase activity